metanephric glomerular epithelial cell differentiation [GO:0072312] (biological process) Definition: The process in which a relatively unspecialized cell acquires specialized features of a metanephric glomerular epithelial cell. Metanephric glomerular epithelial cells are specialized epithelial cells that form part of the metanephric glomerulus; there are two types, metanephric glomerular parietal epithelial cells and metanephric glomerular visceral epithelial cells. Relationships: is a type of cell differentiation involved in metanephros development [GO:0072202]; is a type of GO:0072311; is part of metanephric glomerular epithelium development [GO:0072244] Sources: GOC:mtg_kidney_jan10 Subtypes: metanephric glomerular parietal epithelial cell differentiation [GO:0072245], GO:0072248